{
  "gene": "UniProtKB:Q96RR4",
  "gene_name": "Calcium_calmodulin-dependent protein kinase kinase 2",
  "term_label": "Unknown cellular component",
  "gene_symbol": "CAMKK2",
  "term_id": "UNKNOWN:0003"
}